{
  "gene_symbol": "BRD3OS",
  "term_id": "UNKNOWN:0003",
  "gene_name": "Putative uncharacterized protein BRD3OS",
  "gene": "UniProtKB:A0A1B0GUI7",
  "term_label": "Unknown cellular component"
}